{
  "term_label": "Unknown biological process",
  "gene": "UniProtKB:Q0P5P2",
  "gene_symbol": "C17orf67",
  "gene_name": "Uncharacterized protein C17orf67",
  "term_id": "UNKNOWN:0002"
}